{
  "gene": "UniProtKB:Q96SB8",
  "term_id": "GO:0003684",
  "term_label": "damaged DNA binding",
  "gene_name": "Structural maintenance of chromosomes protein 6",
  "gene_symbol": "SMC6"
}